{
  "gene_name": "Receptor-type tyrosine-protein phosphatase gamma",
  "gene_symbol": "PTPRG",
  "gene": "UniProtKB:P23470",
  "term_label": "Unknown cellular component",
  "term_id": "UNKNOWN:0003"
}